regulation of G0 to G1 transition [GO:0070316] (biological process) Definition: A cell cycle process that modulates the rate or extent of the transition from the G0 quiescent state to the G1 phase. Sources: GOC:mah Relationships: is a type of regulation of cell cycle process [GO:0010564]; regulates G0 to G1 transition [GO:0045023] Subtypes: GO:0070317, positive regulation of G0 to G1 transition [GO:0070318]